{
  "gene": "UniProtKB:Q8N884",
  "term_id": "GO:0005634",
  "term_label": "nucleus",
  "gene_name": "Cyclic GMP-AMP synthase",
  "gene_symbol": "CGAS"
}